pyridoxal phosphate transport [GO:0031921] (biological process) Sources: GOC:mah Relationships: is a type of organic anion transport [GO:0015711]; is a type of organophosphate ester transport [GO:0015748]; is a type of organic hydroxy compound transport [GO:0015850]; is a type of GO:0031919 Definition: The directed movement of pyridoxal phosphate into, out of or within a cell, or between cells, by means of some agent such as a transporter or pore; pyridoxal phosphate is pyridoxal phosphorylated at the hydroxymethyl group of C-5, and is the active form of vitamin B6.